{
  "gene_symbol": "AHR",
  "term_id": "GO:0034751",
  "gene": "UniProtKB:P35869",
  "term_label": "aryl hydrocarbon receptor complex",
  "gene_name": "Aryl hydrocarbon receptor"
}